{
  "term_label": "blood coagulation",
  "gene_symbol": "F5",
  "gene_name": "Coagulation factor V",
  "term_id": "GO:0007596",
  "gene": "UniProtKB:P12259"
}